{
  "gene": "UniProtKB:P53674",
  "term_label": "structural constituent of eye lens",
  "gene_symbol": "CRYBB1",
  "term_id": "GO:0005212",
  "gene_name": "Beta-crystallin B1"
}